regulation of nitric oxide mediated signal transduction [GO:0010749] (biological process) Relationships: is a type of regulation of intracellular signal transduction [GO:1902531]; RO_0002211 nitric oxide mediated signal transduction [GO:0007263] Sources: GOC:BHF, GOC:dph, GOC:tb Also known as: regulation of nitric oxide-mediated signal transduction Definition: Any process that modulates the rate, frequency or extent of nitric oxide mediated signal transduction. Nitric oxide mediated signal transduction is The series of molecular signals mediated by the detection of nitric oxide (NO). Subtypes: positive regulation of nitric oxide mediated signal transduction [GO:0010750], GO:0010751, GO:0141149